muscle alpha-actinin binding [GO:0051371] (molecular function) Also known as: alpha-actinin 2 binding, alpha-actinin 3 binding Relationships: is a type of alpha-actinin binding [GO:0051393] References: PMID:10984498, PMID:11699871, PMID:15014165 Definition: Binding to muscle isoforms of actinin. Muscle alpha-actinin isoforms are found in skeletal and cardiac muscle and are localized to the Z-disc.